regulation of response to amylopectin [GO:1900521] (biological process) Definition: Any process that modulates the frequency, rate or extent of response to amylopectin. Sources: GOC:TermGenie, GOC:mengo_curators Relationships: is a type of regulation of response to stimulus [GO:0048583]; regulates response to amylopectin [GO:0044591] Subtypes: negative regulation of response to amylopectin [GO:1900522], GO:1900523